{
  "gene": "UniProtKB:Q96AM1",
  "gene_symbol": "MRGPRF",
  "term_label": "G protein-coupled receptor signaling pathway",
  "term_id": "GO:0007186",
  "gene_name": "Mas-related G-protein coupled receptor member F"
}